{
  "term_label": "nucleus",
  "term_id": "GO:0005634",
  "gene_symbol": "MPLKIP",
  "gene_name": "M-phase-specific PLK1-interacting protein",
  "gene": "UniProtKB:Q8TAP9"
}